coumarin metabolic process [GO:0009804] (biological process) Relationships: is a type of phenylpropanoid metabolic process [GO:0009698] Sources: GOC:lr, GOC:yl Also known as: coumarin metabolism Definition: The chemical reactions and pathways involving coumarins, compounds derived from the phenylacrylic skeleton of cinnamic acids. Subtypes: GO:0009805, GO:0046226